{
  "gene_name": "Amyloid beta precursor protein binding family B member 1",
  "gene": "UniProtKB:O00213",
  "gene_symbol": "APBB1",
  "term_id": "GO:0060090",
  "term_label": "molecular adaptor activity"
}